pouch outgrowth involved in semicircular canal formation [GO:0060878] (biological process) Definition: The morphogenetic process in which an epithelial sheet bends along a linear axis and gives rise to a pouch that will form a semicircular canal. Relationships: is a type of GO:0048598; is a type of morphogenesis of an epithelial fold [GO:0060571]; is part of semicircular canal formation [GO:0060876] Sources: GOC:dph, GOC:sdb_2009, GOC:tb